disruption of anatomical structure in another organism [GO:0141060] (biological process) Subtypes: symbiont-mediated disruption of host anatomical structure [GO:0052111], venom-mediated disruption of anatomical structure in another organism [GO:0140138], disruption of cellular anatomical structure in another organism [GO:0140975], GO:0141061 Sources: GOC:pg Relationships: is a type of GO:0044419 Definition: The disruption of an anatomical structure of another organism, leading to damage or temporary subversion of that structure.